{
  "term_label": "DNA repair",
  "term_id": "GO:0006281",
  "gene_symbol": "DDB2",
  "gene": "UniProtKB:Q92466",
  "gene_name": "DNA damage-binding protein 2"
}